RISC complex [GO:0016442] (CC) Definition: A ribonucleoprotein complex that contains members of the Argonaute family of proteins, small interfering RNAs (siRNAs) or microRNAs (miRNAs), and miRNA or siRNA-complementary mRNAs, in addition to a number of accessory factors. The RISC complex is involved in posttranscriptional repression of gene expression through downregulation of translation or induction of mRNA degradation. Also known as: RNA-induced silencing complex, miRNP complex, micro-ribonucleoprotein complex Relationships: is a type of RNAi effector complex [GO:0031332] References: PMID:10749213, PMID:15145345